{
  "term_id": "GO:0016324",
  "gene_symbol": "SLC17A1",
  "gene": "UniProtKB:Q14916",
  "gene_name": "Sodium-dependent phosphate transport protein 1",
  "term_label": "apical plasma membrane"
}